{
  "gene": "UniProtKB:O00327",
  "term_label": "nucleus",
  "gene_symbol": "BMAL1",
  "gene_name": "Basic helix-loop-helix ARNT-like protein 1",
  "term_id": "GO:0005634"
}